{
  "term_label": "transforming growth factor beta receptor signaling pathway",
  "gene_name": "Transforming growth factor beta activator LRRC33",
  "gene": "UniProtKB:Q86YC3",
  "term_id": "GO:0007179",
  "gene_symbol": "NRROS"
}